{
  "term_label": "peptidyl-prolyl cis-trans isomerase activity",
  "gene": "UniProtKB:P30414",
  "gene_name": "NK-tumor recognition protein",
  "gene_symbol": "NKTR",
  "term_id": "GO:0003755"
}